{
  "gene_name": "cAMP-dependent protein kinase catalytic subunit PRKX",
  "term_label": "cell adhesion",
  "gene": "UniProtKB:P51817",
  "term_id": "GO:0007155",
  "gene_symbol": "PRKX"
}